{
  "gene": "UniProtKB:Q9BSG1",
  "term_label": "Unknown biological process",
  "gene_name": "Zinc finger protein 2",
  "gene_symbol": "ZNF2",
  "term_id": "UNKNOWN:0002"
}